{
  "term_label": "epidermal growth factor receptor signaling pathway",
  "gene_symbol": "ABL1",
  "gene": "UniProtKB:P00519",
  "term_id": "GO:0007173",
  "gene_name": "Tyrosine-protein kinase ABL1"
}